{
  "gene_name": "Spermatogenesis-associated protein 24",
  "term_label": "nucleus",
  "term_id": "GO:0005634",
  "gene": "UniProtKB:Q86W54",
  "gene_symbol": "SPATA24"
}